{
  "gene": "UniProtKB:Q9UKZ1",
  "term_id": "UNKNOWN:0002",
  "gene_symbol": "CNOT11",
  "term_label": "Unknown biological process",
  "gene_name": "CCR4-NOT transcription complex subunit 11"
}